{
  "gene_symbol": "SSTR5",
  "term_id": "GO:0050796",
  "term_label": "regulation of insulin secretion",
  "gene_name": "Somatostatin receptor type 5",
  "gene": "UniProtKB:P35346"
}